exocytic process [GO:0140029] (biological process) Sources: Wikipedia:Exocytosis Relationships: is a type of cellular process [GO:0009987]; is part of GO:0006887 Subtypes: GO:0001927, serotonin secretion by mast cell [GO:0002552], histamine secretion by mast cell [GO:0002553], serotonin secretion by platelet [GO:0002554], GO:0002555, serotonin secretion by basophil [GO:0002556], histamine secretion by basophil [GO:0002557], vesicle docking involved in exocytosis [GO:0006904], synaptic vesicle targeting [GO:0016080], synaptic vesicle priming [GO:0016082], dense core granule priming [GO:0061789], GO:0070560, vesicle tethering involved in exocytosis [GO:0090522], GO:0099500, pore formation during contractile vacuole discharge [GO:0140028] Definition: The cellular processes that contribute to exocytosis.